{
  "gene": "UniProtKB:P0DMQ5",
  "term_id": "UNKNOWN:0002",
  "gene_name": "Putative transmembrane protein INAFM2",
  "gene_symbol": "INAFM2",
  "term_label": "Unknown biological process"
}